{
  "gene": "UniProtKB:Q6ZV70",
  "term_label": "Unknown cellular component",
  "term_id": "UNKNOWN:0003",
  "gene_symbol": "LANCL3",
  "gene_name": "LanC-like protein 3"
}